{
  "gene_name": "HMG domain-containing protein 4",
  "gene_symbol": "HMGXB4",
  "gene": "UniProtKB:Q9UGU5",
  "term_id": "UNKNOWN:0001",
  "term_label": "Unknown molecular function"
}